{
  "gene_name": "Phytanoyl-CoA hydroxylase-interacting protein-like",
  "term_label": "Unknown molecular function",
  "gene_symbol": "PHYHIPL",
  "gene": "UniProtKB:Q96FC7",
  "term_id": "UNKNOWN:0001"
}